{
  "term_id": "GO:0005813",
  "gene": "UniProtKB:Q16584",
  "term_label": "centrosome",
  "gene_symbol": "MAP3K11",
  "gene_name": "Mitogen-activated protein kinase kinase kinase 11"
}